{
  "term_label": "enzyme inhibitor activity",
  "gene_name": "UDP-glucuronosyltransferase 1A7",
  "term_id": "GO:0004857",
  "gene": "UniProtKB:Q9HAW7",
  "gene_symbol": "UGT1A7"
}